ABC-type bile acid transporter activity [GO:0015432] (molecular function) Relationships: is a type of bile acid transmembrane transporter activity [GO:0015125]; is a type of ATPase-coupled monocarboxylic acid transmembrane transporter activity [GO:0033285]; is a type of ATPase-coupled lipid transmembrane transporter activity [GO:0034040]; is a type of ABC-type transporter activity [GO:0140359] Definition: Enables the transfer of a solute or solutes from one side of a membrane to the other according to the reaction: cholate(in) + ATP + H2O = cholate(out) + ADP + phosphate + H+. Also known as: bile acid porter activity, bile acid-exporting ATPase activity, ATP-dependent bile acid transmembrane transporter activity, ATPase-coupled bile acid transmembrane transporter activity Sources: RHEA:50048